{
  "term_id": "GO:0005737",
  "term_label": "cytoplasm",
  "gene_symbol": "LGSN",
  "gene_name": "Lengsin",
  "gene": "UniProtKB:Q5TDP6"
}